{
  "gene_name": "Meiosis initiator protein",
  "term_label": "Unknown biological process",
  "gene": "UniProtKB:C9JSJ3",
  "gene_symbol": "MEIOSIN",
  "term_id": "UNKNOWN:0002"
}